{
  "gene_name": "Fascin-3",
  "gene": "UniProtKB:Q9NQT6",
  "gene_symbol": "FSCN3",
  "term_id": "GO:0030426",
  "term_label": "growth cone"
}